{
  "gene_symbol": "MICAL2",
  "gene": "UniProtKB:O94851",
  "term_label": "actin cytoskeleton organization",
  "gene_name": "[F-actin]-monooxygenase MICAL2",
  "term_id": "GO:0030036"
}